{
  "term_label": "Unknown molecular function",
  "gene": "UniProtKB:Q9GZR7",
  "gene_name": "ATP-dependent RNA helicase DDX24",
  "term_id": "UNKNOWN:0001",
  "gene_symbol": "DDX24"
}